{
  "gene_symbol": "DSEL",
  "gene": "UniProtKB:Q8IZU8",
  "gene_name": "Dermatan-sulfate epimerase-like protein",
  "term_id": "GO:0050654",
  "term_label": "chondroitin sulfate proteoglycan metabolic process"
}